meiotic spindle astral microtubule [GO:1990574] (cellular component) Definition: Any of the meiotic spindle microtubules that radiate in all directions from the spindle poles and are thought to contribute to the forces that separate the poles and position them in relation to the rest of the cell. Relationships: is a type of astral microtubule [GO:0000235]; is part of meiotic spindle [GO:0072687] References: PMID:10366596